{
  "term_label": "extracellular region",
  "gene_name": "von Willebrand factor D and EGF domain-containing protein",
  "gene": "UniProtKB:Q8N2E2",
  "term_id": "GO:0005576",
  "gene_symbol": "VWDE"
}